{
  "term_label": "protein folding chaperone",
  "gene": "UniProtKB:P34931",
  "gene_name": "Heat shock 70 kDa protein 1-like",
  "gene_symbol": "HSPA1L",
  "term_id": "GO:0044183"
}